{
  "gene_symbol": "ZNF608",
  "gene": "UniProtKB:Q9ULD9",
  "gene_name": "Zinc finger protein 608",
  "term_label": "Unknown molecular function",
  "term_id": "UNKNOWN:0001"
}